{
  "gene_symbol": "ZNF408",
  "term_label": "Unknown cellular component",
  "term_id": "UNKNOWN:0003",
  "gene_name": "Zinc finger protein 408",
  "gene": "UniProtKB:Q9H9D4"
}